cocaine catabolic process [GO:0050784] (biological process) Also known as: cocaine breakdown, cocaine catabolism, cocaine degradation Relationships: is a type of alkaloid catabolic process [GO:0009822] References: PMID:17132243 Definition: The chemical reactions and pathways resulting in the breakdown of cocaine, an alkaloid obtained from the dried leaves of the shrub Erythroxylon coca. It is a cerebral stimulant and narcotic.